{
  "term_id": "GO:0015629",
  "gene": "UniProtKB:Q8N3V7",
  "gene_name": "Synaptopodin",
  "term_label": "actin cytoskeleton",
  "gene_symbol": "SYNPO"
}